glutathione catabolic process [GO:0006751] (biological process) Definition: The chemical reactions and pathways resulting in the breakdown of glutathione, the tripeptide glutamylcysteinylglycine, which acts as a coenzyme for some enzymes and as an antioxidant in the protection of sulfhydryl groups in enzymes and other proteins. Sources: GOC:ai, ISBN:0198506732 Also known as: glutathione breakdown, glutathione catabolism, glutathione degradation Relationships: is a type of glutathione metabolic process [GO:0006749]; is a type of GO:0042219; is a type of sulfur compound catabolic process [GO:0044273]